iron-sulfur cluster export from the mitochondrion [GO:0140466] (biological process) References: PMID:31040179 Relationships: is a type of iron-sulfur cluster transmembrane transport [GO:1902497] Definition: The directed movement of iron sulfur clusters from inside the mitochondrion into the cytosol by crossing the inner mitochondrial membrane.